{
  "gene_symbol": "GRM2",
  "gene": "UniProtKB:Q14416",
  "gene_name": "Metabotropic glutamate receptor 2",
  "term_id": "GO:0051966",
  "term_label": "regulation of synaptic transmission, glutamatergic"
}